{
  "gene": "UniProtKB:P83859",
  "gene_name": "Orexigenic neuropeptide QRFP",
  "term_id": "GO:0005184",
  "gene_symbol": "QRFP",
  "term_label": "neuropeptide hormone activity"
}